{
  "term_id": "GO:0006955",
  "gene_name": "Immunoglobulin kappa variable 1D-17",
  "gene": "UniProtKB:A0A075B6S4",
  "term_label": "immune response",
  "gene_symbol": "IGKV1D-17"
}